vulval cell fate commitment [GO:0072325] (biological process) Relationships: is a type of GO:0045165; is part of vulval development [GO:0040025] References: PMID:11236714 Sources: GOC:kmv, GOC:mah, ISBN:087969307X Definition: The process in which the cellular identity of nematode vulval cells is acquired and determined. In nematodes, the vulva is formed from ventral epidermal cells during larval stages to give rise to a fully formed adult vulva, which is the egg-laying organ of female and hermaphrodite nematodes.